chemokine (C-C motif) ligand 19 production [GO:0097388] (biological process) Relationships: is a type of chemokine production [GO:0032602] Sources: GOC:rv Also known as: CCL19 production, EBI1 ligand chemokine production, ELC production, MIP-3-beta production, macrophage inflammatory protein-3-beta production Definition: The appearance of chemokine (C-C motif) ligand 19 (CCL19) due to biosynthesis or secretion following a cellular stimulus, resulting in an increase in its intracellular or extracellular levels.